{
  "gene_name": "Sialic acid-binding Ig-like lectin 14",
  "term_label": "sialic acid binding",
  "term_id": "GO:0033691",
  "gene_symbol": "SIGLEC14",
  "gene": "UniProtKB:Q08ET2"
}